octadecene biosynthetic process [GO:1900682] (biological process) Sources: GOC:TermGenie, GOC:mengo_curators Regulation: RO_0002211 by GO:1900914; negatively regulated by negative regulation of octadecene biosynthetic process [GO:1900915]; positively regulated by GO:1900916 Relationships: is a type of alkene biosynthetic process [GO:0043450]; is a type of GO:1900681 Also known as: 1-octadecene biosynthetic process, octadecene anabolism, octadecene biosynthesis, octadecene formation, octadecene synthesis Definition: The chemical reactions and pathways resulting in the formation of octadecene.